{
  "gene_symbol": "SELP",
  "gene": "UniProtKB:P16109",
  "term_id": "GO:0009897",
  "term_label": "external side of plasma membrane",
  "gene_name": "P-selectin"
}